{
  "term_id": "GO:0071006",
  "gene": "UniProtKB:Q9BW85",
  "term_label": "U2-type catalytic step 1 spliceosome",
  "gene_symbol": "YJU2",
  "gene_name": "Splicing factor YJU2"
}